{
  "gene_name": "Interleukin-18",
  "gene_symbol": "IL18",
  "gene": "UniProtKB:Q14116",
  "term_id": "GO:0071222",
  "term_label": "cellular response to lipopolysaccharide"
}